{
  "term_label": "regulation of transcription by RNA polymerase II",
  "gene": "UniProtKB:Q5TKA1",
  "gene_symbol": "LIN9",
  "term_id": "GO:0006357",
  "gene_name": "Protein lin-9 homolog"
}